{
  "term_id": "UNKNOWN:0002",
  "gene": "UniProtKB:A0A6Q8PHR7",
  "term_label": "Unknown biological process",
  "gene_symbol": "A0A6Q8PHR7",
  "gene_name": "Uncharacterized protein"
}